{
  "term_label": "Unknown molecular function",
  "term_id": "UNKNOWN:0001",
  "gene_name": "Glycosylphosphatidylinositol anchor attachment 1 protein",
  "gene": "UniProtKB:O43292",
  "gene_symbol": "GPAA1"
}